{
  "gene_name": "Small integral membrane protein 9",
  "term_label": "Unknown molecular function",
  "gene": "UniProtKB:A6NGZ8",
  "term_id": "UNKNOWN:0001",
  "gene_symbol": "SMIM9"
}